{
  "gene_name": "Cadherin-7",
  "gene_symbol": "CDH7",
  "term_label": "adherens junction organization",
  "gene": "UniProtKB:Q9ULB5",
  "term_id": "GO:0034332"
}